{
  "gene": "UniProtKB:Q92734",
  "term_id": "GO:0070971",
  "term_label": "endoplasmic reticulum exit site",
  "gene_symbol": "TFG",
  "gene_name": "Protein TFG"
}